adaptive thermogenesis [GO:1990845] (biological process) References: PMID:17260010, PMID:20363363 Relationships: is a type of metabolic process [GO:0008152] Subtypes: GO:0002024, cold-induced thermogenesis [GO:0106106] Definition: The regulated production of heat in response to short term environmental changes, such as stress, diet or reduced temperature.